{
  "term_label": "ubiquitin-dependent protein catabolic process",
  "gene_name": "RING-box protein 2",
  "gene_symbol": "RNF7",
  "gene": "UniProtKB:Q9UBF6",
  "term_id": "GO:0006511"
}